peptidyl-arginine methylation [GO:0018216] (biological process) Sources: GOC:mah Subtypes: peptidyl-arginine N-methylation [GO:0035246] Relationships: is a type of protein methylation [GO:0006479]; is a type of peptidyl-arginine modification [GO:0018195] Definition: The addition of a methyl group to an arginine residue in a protein.